{
  "term_label": "cell surface",
  "gene_name": "Dendritic cell-specific transmembrane protein",
  "term_id": "GO:0009986",
  "gene": "UniProtKB:Q9H295",
  "gene_symbol": "DCSTAMP"
}